cell adhesion involved in heart morphogenesis [GO:0061343] (biological process) Regulation: regulated by regulation of cell adhesion involved in heart morphogenesis [GO:0061344] Subtypes: endocardial cushion fusion [GO:0003274], cardioblast cell midline fusion [GO:0003317] Relationships: is a type of GO:0007155; is part of heart morphogenesis [GO:0003007] Definition: The attachment of a cell, either to another cell or to an underlying substrate such as the extracellular matrix, via cell adhesion molecules that contributes to the shaping of the heart. References: PMID:16860783 Sources: GOC:dph, GOC:mtg_heart